hematophagy [GO:0140106] (biological process) Relationships: is a type of feeding behavior [GO:0007631]; is a type of GO:0044419 Sources: Wikipedia:Hematophagy Definition: A feeding behavior that involves the ingestion of blood. Hematophagous animals have mouth parts and chemical agents for penetrating vascular structures in the skin of hosts. To overcome natural hemostasis, vasoconstriction, inflammation, and pain sensation in the host, hematophagous animals pre-inject chemical substances with anesthetic and/or anticoagulant properties. Also known as: feeding on blood of other organism, injection of substance into other organism during feeding on blood of other organism, taking of blood meal